{
  "term_label": "metaphase chromosome alignment",
  "term_id": "GO:0051310",
  "gene": "UniProtKB:Q8N0Z3",
  "gene_name": "Spindle and centriole-associated protein 1",
  "gene_symbol": "SPICE1"
}